negative regulation of monocyte chemotaxis [GO:0090027] (biological process) Sources: GOC:dph, GOC:tb Definition: Any process that decreases the frequency, rate, or extent of monocyte chemotaxis. Relationships: is a type of GO:0002689; is a type of GO:0071676; is a type of GO:0090025; negatively regulates monocyte chemotaxis [GO:0002548]